regulation of natural killer cell tolerance induction [GO:0002871] (BP) Definition: Any process that modulates the frequency, rate, or extent of natural killer cell tolerance induction. Sources: GOC:add Also known as: regulation of NK cell tolerance induction Relationships: is a type of regulation of tolerance induction [GO:0002643]; regulates natural killer cell tolerance induction [GO:0002519] Subtypes: negative regulation of natural killer cell tolerance induction [GO:0002872], positive regulation of natural killer cell tolerance induction [GO:0002873]